{
  "term_label": "Unknown cellular component",
  "term_id": "UNKNOWN:0003",
  "gene": "UniProtKB:Q8N2G6",
  "gene_symbol": "ZCCHC24",
  "gene_name": "Zinc finger CCHC domain-containing protein 24"
}